{
  "gene_name": "Protein FAM149A",
  "gene_symbol": "FAM149A",
  "term_label": "Unknown cellular component",
  "term_id": "UNKNOWN:0003",
  "gene": "UniProtKB:A5PLN7"
}